{
  "gene": "UniProtKB:Q96ST8",
  "gene_symbol": "CEP89",
  "term_label": "Unknown molecular function",
  "term_id": "UNKNOWN:0001",
  "gene_name": "Centrosomal protein of 89 kDa"
}